{
  "gene_symbol": "FAIM",
  "term_label": "negative regulation of extrinsic apoptotic signaling pathway via death domain receptors",
  "gene_name": "Fas apoptotic inhibitory molecule 1",
  "term_id": "GO:1902042",
  "gene": "UniProtKB:Q9NVQ4"
}